{
  "term_label": "regulation of RNA splicing",
  "gene_symbol": "CLK1",
  "term_id": "GO:0043484",
  "gene": "UniProtKB:P49759",
  "gene_name": "Dual specificity protein kinase CLK1"
}